{
  "term_id": "GO:0008009",
  "gene_symbol": "CX3CL1",
  "gene_name": "Fractalkine",
  "gene": "UniProtKB:P78423",
  "term_label": "chemokine activity"
}